synaptic signaling by nitric oxide [GO:0099163] (biological process) References: PMID:19038221 Sources: GOC:dos Regulation: regulated by regulation of synaptic signaling by nitric oxide [GO:0150045] Definition: Cell-cell signaling to or from a synapse, mediated by nitric oxide. Subtypes: trans-synaptic signaling by nitric oxide [GO:0099548] Relationships: is a type of synaptic signaling [GO:0099536]